G protein-coupled folate receptor activity [GO:0106063] (molecular function) Also known as: G-protein coupled folate receptor activity, G-protein coupled folic acid receptor activity Definition: Combining with folate and transmitting the signal from one side of the membrane to the other by activating an associated G-protein, initiating a change in cell activity. References: PMID:26906738 Relationships: is a type of G protein-coupled receptor activity [GO:0004930]